Ran protein signal transduction [GO:0031291] (BP) Sources: GOC:mah Definition: An intracellular signaling cassette in which a small monomeric GTPase of the Ran subfamily relays a signal. Relationships: is a type of small GTPase-mediated signal transduction [GO:0007264]